{
  "gene_symbol": "PCDHB9",
  "term_id": "GO:0007155",
  "term_label": "cell adhesion",
  "gene_name": "Protocadherin beta-9",
  "gene": "UniProtKB:Q9Y5E1"
}